{
  "gene_symbol": "MC3R",
  "term_id": "GO:0005886",
  "gene_name": "Melanocortin receptor 3",
  "term_label": "plasma membrane",
  "gene": "UniProtKB:P41968"
}